{
  "gene_name": "Interleukin-18-binding protein",
  "term_label": "extracellular space",
  "gene": "UniProtKB:O95998",
  "term_id": "GO:0005615",
  "gene_symbol": "IL18BP"
}